micropinocytosis [GO:0044350] (biological process) Also known as: clathrin-independent pinocytosis, single-organism micropinocytosis References: PMID:14731589, PMID:14732047 Definition: An endocytosis process that results in the uptake of liquid material by cells from their external environment by invagination of the plasma membrane to form uncoated micropinosomes, differentiated from macropinosomes by their smaller size, on average 95 nm. Relationships: is a type of pinocytosis [GO:0006907]